{
  "term_id": "GO:0005886",
  "gene_symbol": "OR6T1",
  "term_label": "plasma membrane",
  "gene_name": "Olfactory receptor 6T1",
  "gene": "UniProtKB:Q8NGN1"
}